chloroplast ribulose bisphosphate carboxylase complex [GO:0009573] (cellular component) Definition: A complex, located in the chloroplast, containing either both large and small subunits or just small subunits which carries out the activity of producing 3-phosphoglycerate from carbon dioxide and ribulose-1,5-bisphosphate. An example of this component is found in Arabidopsis thaliana. Relationships: is a type of ribulose bisphosphate carboxylase complex [GO:0048492]; is part of chloroplast stroma [GO:0009570] Also known as: chloroplast RubisCO complex Sources: GOC:mlg, GOC:mtg_sensu